4-carboxymethyl-4-methylbutenolide mutase activity [GO:0047469] (molecular function) Relationships: is a type of GO:0016866 Also known as: 4-carboxymethyl-4-methylbut-2-en-1,4-olide methylmutase activity, 4-methyl-2-enelactone isomerase activity, 4-methyl-2-enelactone methyl-isomerase activity, 4-methyl-3-enelactone methyl isomerase activity, 4-methylmuconolactone methylisomerase activity Sources: EC:5.4.99.14, RHEA:19237 Definition: Catalysis of the reaction: 4-carboxymethyl-4-methylbut-2-en-1,4-olide = 4-carboxymethyl-3-methylbut-2-en-1,4-olide.